protein localization to Golgi apparatus [GO:0034067] (biological process) Definition: A process in which a protein is transported to, or maintained in, a location within the Golgi apparatus. Subtypes: protein localization to ERGIC [GO:0106272], protein localization to Golgi membrane [GO:1903292] Relationships: is a type of GO:0033365 Also known as: protein localisation in Golgi apparatus, protein localization in Golgi apparatus, establishment of protein localisation to Golgi, establishment of protein localization in Golgi, establishment of protein localization to Golgi, establishment of protein localization to Golgi apparatus, protein targeting to Golgi, protein-Golgi targeting Sources: GOC:mah